{
  "gene_name": "Chromodomain-helicase-DNA-binding protein 1",
  "gene": "UniProtKB:O14646",
  "gene_symbol": "CHD1",
  "term_id": "GO:0005634",
  "term_label": "nucleus"
}